{
  "gene_name": "Low molecular weight phosphotyrosine protein phosphatase",
  "term_id": "GO:0004725",
  "gene_symbol": "ACP1",
  "term_label": "protein tyrosine phosphatase activity",
  "gene": "UniProtKB:P24666"
}